snRNP binding [GO:0070990] (molecular function) Sources: GOC:BHF, GOC:mah, GOC:rl Relationships: is a type of ribonucleoprotein complex binding [GO:0043021] Definition: Binding to a small nuclear ribonucleoprotein particle. Subtypes: U1 snRNP binding [GO:1990446], U2 snRNP binding [GO:1990447]